external side of cell wall [GO:0010339] (cellular component) Definition: The side of the cell wall that is opposite to the side that faces the cell and its contents. Relationships: is a type of cellular anatomical structure [GO:0110165]; is part of GO:0005618; is part of GO:0009986 Subtypes: external side of fungal-type cell wall [GO:0070263] Sources: GOC:mtg_sensu, GOC:tb